regulation of actin filament length [GO:0030832] (biological process) Subtypes: regulation of actin polymerization or depolymerization [GO:0008064] Note: Note that the syntax of the definition of this term is different from the usual regulation syntax because it describes regulation of a trait rather than regulation of a process. Sources: GOC:dph, GOC:mah Definition: Any process that controls the length of actin filaments in a cell. Relationships: is a type of regulation of cellular component size [GO:0032535]; is a type of regulation of actin cytoskeleton organization [GO:0032956]